{
  "gene": "UniProtKB:Q01201",
  "term_id": "GO:0045944",
  "gene_symbol": "RELB",
  "gene_name": "Transcription factor RelB",
  "term_label": "positive regulation of transcription by RNA polymerase II"
}